{
  "gene_symbol": "HOOK2",
  "gene": "UniProtKB:Q96ED9",
  "gene_name": "Protein Hook homolog 2",
  "term_id": "GO:0031122",
  "term_label": "cytoplasmic microtubule organization"
}